{
  "gene_name": "Homeobox protein Hox-D8",
  "gene": "UniProtKB:P13378",
  "gene_symbol": "HOXD8",
  "term_id": "GO:0006357",
  "term_label": "regulation of transcription by RNA polymerase II"
}